{
  "term_label": "sperm midpiece",
  "gene_symbol": "TACR2",
  "gene": "UniProtKB:P21452",
  "term_id": "GO:0097225",
  "gene_name": "Substance-K receptor"
}